{
  "gene_name": "Vinexin",
  "term_id": "GO:0031589",
  "term_label": "cell-substrate adhesion",
  "gene_symbol": "SORBS3",
  "gene": "UniProtKB:O60504"
}